{
  "term_label": "endoplasmic reticulum",
  "gene_symbol": "PRKN",
  "term_id": "GO:0005783",
  "gene_name": "E3 ubiquitin-protein ligase parkin",
  "gene": "UniProtKB:O60260"
}